{
  "term_label": "myosin phosphatase regulator activity",
  "gene": "UniProtKB:O60237",
  "gene_name": "Protein phosphatase 1 regulatory subunit 12B",
  "gene_symbol": "PPP1R12B",
  "term_id": "GO:0017020"
}